{
  "gene_symbol": "SLITRK4",
  "term_label": "positive regulation of synapse assembly",
  "term_id": "GO:0051965",
  "gene": "UniProtKB:Q8IW52",
  "gene_name": "SLIT and NTRK-like protein 4"
}